{
  "gene_symbol": "HTR2B",
  "term_label": "neurotransmitter receptor activity",
  "gene": "UniProtKB:P41595",
  "term_id": "GO:0030594",
  "gene_name": "5-hydroxytryptamine receptor 2B"
}